{
  "gene_name": "Palmitoyltransferase ZDHHC8",
  "term_label": "palmitoyltransferase activity",
  "gene": "UniProtKB:Q9ULC8",
  "term_id": "GO:0016409",
  "gene_symbol": "ZDHHC8"
}